{
  "term_label": "proton-transporting ATP synthase complex",
  "term_id": "GO:0045259",
  "gene_name": "ATP synthase F(0) complex subunit C2, mitochondrial",
  "gene": "UniProtKB:Q06055",
  "gene_symbol": "ATP5MC2"
}